oxidoreductase activity, acting on hydrogen as donor, iron-sulfur protein as acceptor [GO:0016699] (molecular function) Also known as: oxidoreductase activity, acting on hydrogen as donor, iron-sulphur protein as acceptor Relationships: is a type of oxidoreductase activity, acting on hydrogen as donor [GO:0016695] Sources: GOC:jl Definition: Catalysis of an oxidation-reduction (redox) reaction in which hydrogen acts as an electron donor and reduces an iron-sulfur protein. Subtypes: ferredoxin hydrogenase activity [GO:0008901]